{
  "term_id": "UNKNOWN:0003",
  "gene": "UniProtKB:Q309B1",
  "term_label": "Unknown cellular component",
  "gene_symbol": "TRIM16L",
  "gene_name": "Tripartite motif-containing protein 16-like protein"
}